{
  "gene": "UniProtKB:Q9NRC1",
  "term_label": "Unknown cellular component",
  "gene_symbol": "ST7",
  "term_id": "UNKNOWN:0003",
  "gene_name": "Suppressor of tumorigenicity 7 protein"
}